all-trans-decaprenyl-diphosphate synthase activity [GO:0097269] (molecular function) Definition: Catalysis of the reaction: 7 isopentenyl diphosphate + (2E,6E)-farnesyl diphosphate = all-trans-decaprenyl diphosphate + 7 diphosphate. Relationships: is a type of GO:0120531 References: PMID:16262699 Sources: RHEA:27802 Also known as: decaprenyl pyrophosphate synthetase activity, decaprenyl-diphosphate synthase activity, polyprenylpyrophosphate synthetase activity, terpenoidallyltransferase activity, terpenyl pyrophosphate synthetase activity, trans-prenyltransferase activity, (2E,6E)-farnesyl-diphosphate:isopentenyl-diphosphate farnesyltranstransferase activity, 2-trans,6-trans-farnesyl diphosphate activity